{
  "gene_name": "Putative protein PRAC2",
  "term_id": "UNKNOWN:0001",
  "gene": "UniProtKB:D3DTV9",
  "term_label": "Unknown molecular function",
  "gene_symbol": "PRAC2"
}